{
  "gene": "UniProtKB:P43115",
  "gene_name": "Prostaglandin E2 receptor EP3 subtype",
  "gene_symbol": "PTGER3",
  "term_id": "GO:0004957",
  "term_label": "prostaglandin E receptor activity"
}